{
  "gene_symbol": "SLC25A31",
  "gene_name": "ADP_ATP translocase 4",
  "term_id": "GO:1990544",
  "term_label": "mitochondrial ATP transmembrane transport",
  "gene": "UniProtKB:Q9H0C2"
}